baculum development [GO:1990375] (biological process) Relationships: is_a reproductive structure development [GO:0048608] Also known as: os penis development, penile bone development, penis bone development Definition: The reproductive developmental process whose specific outcome is the progression of the baculum over time, from its formation to the mature structure. References: PMID:21471296 Sources: GOC:sl